{
  "gene_name": "Small ribosomal subunit protein eS7",
  "gene": "UniProtKB:P62081",
  "term_label": "small-subunit processome",
  "term_id": "GO:0032040",
  "gene_symbol": "RPS7"
}